exine [GO:0043668] (CC) Note: Note that the exine is highly resistant to strong acids and bases. Definition: The outer layer of the pollen grain wall which is composed primarily of sporopollenin. Sources: https://doi.org/10.1038/220389a0 Relationships: is a type of GO:0110165; is part of pollen wall [GO:0043667]